{
  "term_id": "GO:0005634",
  "gene": "UniProtKB:A6NFI3",
  "gene_name": "Zinc finger protein 316",
  "gene_symbol": "ZNF316",
  "term_label": "nucleus"
}